rhombomere 6 development [GO:0021572] (biological process) Definition: The process whose specific outcome is the progression of rhombomere 6 over time, from its formation to the mature structure. Rhombomeres are transverse segments of the developing rhombencephalon. Rhombomeres are lineage restricted, express different genes from one another, and adopt different developmental fates. Rhombomeres are numbered in anterior to posterior order. Sources: GOC:cls, GOC:curators, GOC:dgh, GOC:dph, GOC:jid Relationships: is a type of rhombomere development [GO:0021546]